negative regulation of podosome assembly [GO:0071802] (biological process) Definition: Any process that stops, prevents or reduces the rate or extent of podosome assembly. Relationships: is a type of GO:0031333; is a type of GO:0071801; is a type of GO:1902116; negatively regulates podosome assembly [GO:0071800] Also known as: down regulation of podosome assembly, down-regulation of podosome assembly, downregulation of podosome assembly, inhibition of podosome assembly Sources: GOC:mah, GOC:sl